{
  "gene": "UniProtKB:Q9Y6N6",
  "term_id": "GO:0005615",
  "gene_name": "Laminin subunit gamma-3",
  "gene_symbol": "LAMC3",
  "term_label": "extracellular space"
}